{
  "term_id": "GO:0050262",
  "gene_name": "Nicotinamide riboside kinase 1",
  "gene_symbol": "NMRK1",
  "gene": "UniProtKB:Q9NWW6",
  "term_label": "ribosylnicotinamide kinase activity"
}